spinal cord oligodendrocyte cell fate specification [GO:0021530] (biological process) Definition: The process in which a cell becomes capable of differentiating autonomously into an oligodendrocyte in an environment that is neutral with respect to the developmental pathway. Sources: GOC:cls, GOC:dgh, GOC:dph, GOC:jid, GO_REF:0000021 Relationships: is_a oligodendrocyte cell fate specification [GO:0021778]; is part of spinal cord oligodendrocyte cell differentiation [GO:0021529]